{
  "term_label": "endoplasmic reticulum tubular network",
  "gene": "UniProtKB:Q9H4P4",
  "term_id": "GO:0071782",
  "gene_name": "E3 ubiquitin-protein ligase NRDP1",
  "gene_symbol": "RNF41"
}